{
  "gene_name": "FAD-linked sulfhydryl oxidase ALR",
  "term_label": "mitochondrion",
  "gene_symbol": "GFER",
  "term_id": "GO:0005739",
  "gene": "UniProtKB:P55789"
}